{
  "term_label": "Unknown molecular function",
  "term_id": "UNKNOWN:0001",
  "gene_name": "Uncharacterized protein C6orf47",
  "gene_symbol": "C6orf47",
  "gene": "UniProtKB:O95873"
}